{
  "gene": "UniProtKB:Q99935",
  "term_id": "GO:0051930",
  "term_label": "regulation of sensory perception of pain",
  "gene_name": "Opiorphin prepropeptide",
  "gene_symbol": "OPRPN"
}